proteasome core complex, beta-subunit complex [GO:0019774] (cellular component) References: PMID:10854779 Sources: GOC:jl, GOC:mtg_sensu, GOC:rb Definition: The proteasome core subcomplex that constitutes the two inner rings of the proteasome core complex. An example of this component is found in Mus musculus. Relationships: is a type of protein-containing complex [GO:0032991]; BFO_0000050 intracellular anatomical structure [GO:0005622]; is part of proteasome core complex [GO:0005839] Subtypes: nuclear proteasome core complex, beta-subunit complex [GO:0031607], cytosolic proteasome core complex, beta-subunit complex [GO:0031609]